amide transmembrane transporter activity [GO:0042887] (molecular function) Sources: GOC:jl, ISBN:0198506732 Definition: Enables the transfer of an amide, any compound containing one, two, or three acyl groups attached to a nitrogen atom, from one side of a membrane to the other. Also known as: amine/amide/polyamine channel activity Relationships: is a type of GO:0022857; is part of amide transport [GO:0042886] Subtypes: allantoin:proton symporter activity [GO:0005274], folic acid transmembrane transporter activity [GO:0008517], acetyl-CoA transmembrane transporter activity [GO:0008521], GO:0015124, L-asparagine transmembrane transporter activity [GO:0015182], GO:0015204, biotin transmembrane transporter activity [GO:0015225], coenzyme A transmembrane transporter activity [GO:0015228], GO:0015233, cycloheximide transmembrane transporter activity [GO:0015243], GO:0015306, benomyl:proton antiporter activity [GO:0015310], methotrexate transmembrane transporter activity [GO:0015350], pantothenate:sodium symporter activity [GO:0015498], sulfathiazole transmembrane transporter activity [GO:0015546], ABC-type fatty-acyl-CoA transporter activity [GO:0015607], microcin transmembrane transporter activity [GO:0015638], bacteriocin transmembrane transporter activity [GO:0022885], GO:0035673, chloramphenicol transmembrane transporter activity [GO:0042896], polymyxin transmembrane transporter activity [GO:0042897], fosmidomycin transmembrane transporter activity [GO:0042898], ferrichrome transmembrane transporter activity [GO:0042929], achromobactin transmembrane transporter activity [GO:0042934], GO:0044604, dethiobiotin transmembrane transporter activity [GO:1901604], 5-amino-1-ribofuranosylimidazole-4-carboxamide transmembrane transporter activity [GO:1903089], carcinine transmembrane transporter activity [GO:1905131]